{
  "term_label": "hemopoiesis",
  "gene_symbol": "MEIS3P1",
  "gene": "UniProtKB:A6NDR6",
  "gene_name": "Putative homeobox protein Meis3-like 1",
  "term_id": "GO:0030097"
}